{
  "term_id": "GO:0000785",
  "gene": "UniProtKB:Q9H2G4",
  "term_label": "chromatin",
  "gene_symbol": "TSPYL2",
  "gene_name": "Testis-specific Y-encoded-like protein 2"
}